{
  "gene_symbol": "PRND",
  "gene": "UniProtKB:Q9UKY0",
  "term_label": "plasma membrane",
  "gene_name": "Prion-like protein doppel",
  "term_id": "GO:0005886"
}